{
  "gene": "UniProtKB:Q5SZL2",
  "gene_name": "Centrosomal protein of 85 kDa-like",
  "term_id": "GO:0005813",
  "term_label": "centrosome",
  "gene_symbol": "CEP85L"
}